{
  "term_id": "GO:0015629",
  "term_label": "actin cytoskeleton",
  "gene_symbol": "FLII",
  "gene_name": "Protein flightless-1 homolog",
  "gene": "UniProtKB:Q13045"
}